{
  "gene": "UniProtKB:Q7Z340",
  "gene_name": "Zinc finger protein 551",
  "gene_symbol": "ZNF551",
  "term_label": "RNA polymerase II cis-regulatory region sequence-specific DNA binding",
  "term_id": "GO:0000978"
}